regulation of maintenance of bipolar cell polarity regulating cell shape [GO:2000115] (biological process) Subtypes: positive regulation of maintenance of bipolar cell polarity regulating cell shape [GO:0061361], negative regulation of maintenance of bipolar cell polarity regulating cell shape [GO:0061362] Sources: GOC:obol Definition: Any process that modulates the frequency, rate or extent of maintenance of bipolar cell polarity regulating in cell shape. Relationships: is_a regulation of establishment or maintenance of bipolar cell polarity regulating cell shape [GO:2000100]; regulates maintenance of bipolar cell polarity regulating cell shape [GO:0061305]